{
  "gene_name": "Olfactory receptor 3A1",
  "term_id": "GO:0007165",
  "gene_symbol": "OR3A1",
  "gene": "UniProtKB:P47881",
  "term_label": "signal transduction"
}